{
  "gene_symbol": "HSBP1",
  "term_label": "Unknown molecular function",
  "gene_name": "Heat shock factor-binding protein 1",
  "term_id": "UNKNOWN:0001",
  "gene": "UniProtKB:O75506"
}